DNA transposition [GO:0006313] (biological process) Also known as: Class II transposition, transposition, DNA-mediated Definition: A type of transposition in which a transposable element (transposon) is moved to another part of a genome, either by a cut-and-paste mechanism or a replicative mechanism. Subtypes: non-replicative DNA transposition [GO:0098038], replicative DNA transposition [GO:0098039] References: PMID:26846462, PMID:30416149, PMID:32588192 Sources: ISBN:0198506732, ISBN:1555812090 Relationships: is a type of DNA recombination [GO:0006310]; is a type of transposition [GO:0032196]